glycerone phosphate:phosphate antiporter activity [GO:0051407] (molecular function) Relationships: is a type of organophosphate:phosphate antiporter activity [GO:0015315]; is a type of organophosphate ester transmembrane transporter activity [GO:0015605]; is_a alcohol transmembrane transporter activity [GO:0015665]; is a type of carbohydrate derivative transmembrane transporter activity [GO:1901505] Also known as: dihydroxyacetone-phosphate:inorganic phosphate antiporter activity, glycerone phosphate:inorganic phosphate antiporter activity Definition: Enables the transfer of a solute or solutes from one side of a membrane to the other according to the reaction: glycerone phosphate(out) + phosphate(in) = glycerone phosphate(in) + phosphate(out). Sources: GOC:ai